regulation of chemokine (C-C motif) ligand 1 production [GO:0071652] (biological process) Subtypes: GO:0071653, GO:0071654 Relationships: is a type of regulation of chemokine production [GO:0032642]; regulates chemokine (C-C motif) ligand 1 production [GO:0071610] Sources: GOC:mah Also known as: regulation of CCL1 production, regulation of T cell activation 3 production, regulation of TCA-3 production Definition: Any process that modulates the frequency, rate, or extent of production of chemokine (C-C motif) ligand 1.